{
  "gene": "UniProtKB:P29400",
  "term_label": "collagen type IV trimer",
  "gene_name": "Collagen alpha-5(IV) chain",
  "gene_symbol": "COL4A5",
  "term_id": "GO:0005587"
}